{
  "term_label": "RNA polymerase II cis-regulatory region sequence-specific DNA binding",
  "term_id": "GO:0000978",
  "gene": "UniProtKB:P0CG23",
  "gene_name": "Zinc finger protein 853",
  "gene_symbol": "ZNF853"
}